{
  "gene_symbol": "URI1",
  "term_label": "phosphatase inhibitor activity",
  "gene": "UniProtKB:O94763",
  "gene_name": "Unconventional prefoldin RPB5 interactor 1",
  "term_id": "GO:0019212"
}